{
  "gene_name": "Olfactory receptor 5D13",
  "gene_symbol": "OR5D13",
  "term_label": "Unknown cellular component",
  "gene": "UniProtKB:Q8NGL4",
  "term_id": "UNKNOWN:0003"
}